{
  "term_label": "cytosol",
  "gene_symbol": "XYLB",
  "term_id": "GO:0005829",
  "gene": "UniProtKB:O75191",
  "gene_name": "Xylulose kinase"
}